positive regulation of G2/M transition of mitotic cell cycle involved in cellular response to nitrogen starvation [GO:1905287] (biological process) Also known as: positive regulation of mitotic entry involved in cellular response to nitrogen starvation Relationships: is_a positive regulation of G2/M transition of mitotic cell cycle [GO:0010971]; BFO_0000050 cellular response to nitrogen starvation [GO:0006995] Definition: Any positive regulation of G2/M transition of mitotic cell cycle that is involved in cellular response to nitrogen starvation. References: PMID:26776736 Sources: GOC:TermGenie, GO_REF:0000060